{
  "term_label": "RNA splicing",
  "gene_symbol": "ACIN1",
  "gene_name": "Apoptotic chromatin condensation inducer in the nucleus",
  "gene": "UniProtKB:Q9UKV3",
  "term_id": "GO:0008380"
}